{
  "gene": "UniProtKB:A0A0U1RRA0",
  "gene_name": "Putative transmembrane protein ZNF593OS",
  "term_id": "UNKNOWN:0003",
  "term_label": "Unknown cellular component",
  "gene_symbol": "ZNF593OS"
}